alpha11-beta1 integrin-collagen type I complex [GO:0071087] (cellular component) Relationships: is a type of plasma membrane protein complex [GO:0098797] Definition: A protein complex that consists of an alpha11-beta1 integrin complex bound to a type I collagen. Also known as: ITGA11-ITGB1-COL1A1 complex References: PMID:10464311